{
  "term_label": "cellular response to nitrogen starvation",
  "term_id": "GO:0006995",
  "gene_name": "Microtubule-associated proteins 1A_1B light chain 3A",
  "gene": "UniProtKB:Q9H492",
  "gene_symbol": "MAP1LC3A"
}